3-mercaptopyruvate sulfurtransferase activity [GO:0016784] (MF) Definition: Catalysis of the reaction: 2-oxo-3-sulfanylpropanoate + [thioredoxin]-dithiol = [thioredoxin]-disulfide + hydrogen sulfide + pyruvate + H+. Note that 2-oxo-3-sulfanylpropanoate is also known as 3-mercaptopyruvate. Sources: RHEA:21740 Also known as: 3-mercaptopyruvate sulphurtransferase activity, mercaptopyruvate sulfurtransferase activity, 3-mercaptopyruvate:cyanide sulfurtransferase activity, beta-mercaptopyruvate sulfurtransferase activity Relationships: is a type of sulfurtransferase activity [GO:0016783]